{
  "gene_symbol": "LTN1",
  "term_label": "ribosome-associated ubiquitin-dependent protein catabolic process",
  "gene": "UniProtKB:O94822",
  "term_id": "GO:1990116",
  "gene_name": "E3 ubiquitin-protein ligase listerin"
}